carboxylesterase activity [GO:0106435] (molecular function) Relationships: is a type of carboxylic ester hydrolase activity [GO:0052689] Definition: Catalysis of the reaction: a carboxylic ester + H2O = a carboxylate + an alcohol + H+. Also known as: B-esterase activity, alpha-carboxylesterase activity, cocaine esterase, procaine esterase, serine esterase activity, triacetin esterase, vitamin A esterase, ali-esterase activity, nonspecific carboxylesterase activity Note: Note: This covers a broad range of specificity; also hydrolyzes vitamin A esters. Sources: RHEA:21164